{
  "gene_name": "Putative uncharacterized protein FLJ40606",
  "term_id": "UNKNOWN:0003",
  "gene_symbol": "P0C880",
  "term_label": "Unknown cellular component",
  "gene": "UniProtKB:P0C880"
}